{
  "gene": "UniProtKB:Q5VZB9",
  "gene_name": "Doublesex- and mab-3-related transcription factor A1",
  "gene_symbol": "DMRTA1",
  "term_id": "GO:0006357",
  "term_label": "regulation of transcription by RNA polymerase II"
}